{
  "term_id": "UNKNOWN:0003",
  "gene_symbol": "LRRC43",
  "term_label": "Unknown cellular component",
  "gene_name": "Leucine-rich repeat-containing protein 43",
  "gene": "UniProtKB:Q8N309"
}